{
  "term_id": "UNKNOWN:0002",
  "gene_name": "FERM, ARHGEF and pleckstrin domain-containing protein 2",
  "gene_symbol": "FARP2",
  "gene": "UniProtKB:O94887",
  "term_label": "Unknown biological process"
}